{
  "gene_name": "Zinc finger protein 416",
  "term_label": "RNA polymerase II cis-regulatory region sequence-specific DNA binding",
  "gene_symbol": "ZNF416",
  "term_id": "GO:0000978",
  "gene": "UniProtKB:Q9BWM5"
}